{
  "gene": "UniProtKB:Q3KP31",
  "term_id": "GO:0006357",
  "gene_name": "Zinc finger protein 791",
  "gene_symbol": "ZNF791",
  "term_label": "regulation of transcription by RNA polymerase II"
}